{
  "gene": "UniProtKB:P17516",
  "term_id": "GO:0044597",
  "gene_symbol": "AKR1C4",
  "gene_name": "Aldo-keto reductase family 1 member C4",
  "term_label": "daunorubicin metabolic process"
}